{
  "term_label": "Unknown cellular component",
  "term_id": "UNKNOWN:0003",
  "gene": "UniProtKB:Q8NFX7",
  "gene_symbol": "STXBP6",
  "gene_name": "Syntaxin-binding protein 6"
}